neural crest cell migration involved in sympathetic nervous system development [GO:1903045] (biological process) References: PMID:19325129 Sources: GOC:BHF, GOC:TermGenie, GOC:rl, GO_REF:0000060 Definition: Any neural crest cell migration that is involved in sympathetic nervous system development. Relationships: is a type of neural crest cell migration involved in autonomic nervous system development [GO:1901166]; is part of sympathetic nervous system development [GO:0048485] Note: Sema3a (O08665, mouse) is involved in neural crest cell migration involved in sympathetic nervous system development